{
  "gene_symbol": "CEACAM19",
  "gene_name": "Carcinoembryonic antigen-related cell adhesion molecule 19",
  "term_label": "homophilic cell-cell adhesion",
  "gene": "UniProtKB:Q7Z692",
  "term_id": "GO:0007156"
}